{
  "gene_name": "Zinc finger protein 697",
  "gene": "UniProtKB:Q5TEC3",
  "gene_symbol": "ZNF697",
  "term_id": "GO:0000981",
  "term_label": "DNA-binding transcription factor activity, RNA polymerase II-specific"
}